{
  "gene_name": "Band 4.1-like protein 2",
  "gene_symbol": "EPB41L2",
  "term_id": "GO:0005886",
  "term_label": "plasma membrane",
  "gene": "UniProtKB:O43491"
}